compound eye pigment cell differentiation [GO:0062056] (biological process) Definition: The process in which a relatively unspecialized cell acquires the specialized features of a compound eye pigment cell, a cell of the retina containing screening pigments that functions to screen photoreceptors from light leaking from adjacent ommatidia. Relationships: is_a pigment cell differentiation [GO:0050931]; is part of compound eye morphogenesis [GO:0001745] References: PMID:8929534 Sources: GOC:ha